negative regulation of purine nucleotide metabolic process [GO:1900543] (biological process) Subtypes: negative regulation of purine nucleotide catabolic process [GO:0033122], GO:1900372, GO:1902689, negative regulation of ATP metabolic process [GO:1903579], negative regulation of pentose-phosphate shunt [GO:1905856] Relationships: is a type of negative regulation of nucleotide metabolic process [GO:0045980]; is a type of GO:1900542; negatively regulates purine nucleotide metabolic process [GO:0006163] Also known as: down regulation of purine nucleotide metabolic process, down regulation of purine nucleotide metabolism, down-regulation of purine nucleotide metabolic process, down-regulation of purine nucleotide metabolism, downregulation of purine nucleotide metabolic process, downregulation of purine nucleotide metabolism, negative regulation of purine nucleotide metabolism, down regulation of purine metabolic process, down regulation of purine metabolism, down-regulation of purine metabolic process, down-regulation of purine metabolism, downregulation of purine metabolic process, downregulation of purine metabolism, inhibition of purine metabolic process, inhibition of purine metabolism, inhibition of purine nucleotide metabolic process, inhibition of purine nucleotide metabolism, negative regulation of purine metabolic process, negative regulation of purine metabolism Sources: GOC:TermGenie Definition: Any process that stops, prevents or reduces the frequency, rate or extent of purine nucleotide metabolic process.